{
  "term_id": "GO:0005886",
  "term_label": "plasma membrane",
  "gene_symbol": "SLC35G1",
  "gene_name": "Solute carrier family 35 member G1",
  "gene": "UniProtKB:Q2M3R5"
}